ferric triacetylfusarinine C transmembrane transporter activity [GO:0015621] (molecular function) Relationships: is a type of transmembrane transporter activity [GO:0022857] Subtypes: GO:0015346 Sources: GOC:ai Definition: Enables the transfer of ferric triacetylfusarinine C from one side of a membrane to the other.